melanocyte-stimulating hormone receptor activity [GO:0004980] (molecular function) Also known as: MSH receptor activity, MSHR activity, melanocyte stimulating hormone receptor activity, melanophore-stimulating hormone receptor activity References: PMID:7581459 Sources: GOC:jl Relationships: is a type of GO:0004977; has part hormone binding [GO:0042562] Definition: Combining with melanocyte-stimulating hormone to initiate a change in cell activity.